negative regulation of establishment of blood-brain barrier [GO:0090212] (biological process) Sources: GOC:dph, GOC:tb Also known as: negative regulation of establishment of BBB Definition: Any process that decreases the rate, frequency or extent of the establishment of the blood-brain barrier, a selectively permeable structural and functional barrier that exists between the capillaries and the brain. Relationships: is a type of negative regulation of cell development [GO:0010721]; is a type of GO:0090210; negatively regulates establishment of blood-brain barrier [GO:0060856]